positive regulation of synaptic plasticity [GO:0031915] (BP) Relationships: is a type of GO:0048167 Definition: A process that increases synaptic plasticity, the ability of synapses to change as circumstances require. They may alter function, such as increasing or decreasing their sensitivity, or they may increase or decrease in actual numbers. Sources: GOC:mah Subtypes: positive regulation of synaptic metaplasticity [GO:0031918], positive regulation of synaptic plasticity by chemical substance [GO:0051914] Also known as: up regulation of synaptic plasticity, up-regulation of synaptic plasticity, upregulation of synaptic plasticity, activation of synaptic plasticity, stimulation of synaptic plasticity